{
  "gene_name": "Metallothionein-1F",
  "term_id": "GO:0071294",
  "gene": "UniProtKB:P04733",
  "term_label": "cellular response to zinc ion",
  "gene_symbol": "MT1F"
}